{
  "term_id": "GO:0005654",
  "gene": "UniProtKB:Q9Y2K1",
  "gene_name": "Zinc finger and BTB domain-containing protein 1",
  "gene_symbol": "ZBTB1",
  "term_label": "nucleoplasm"
}